{
  "gene": "UniProtKB:A0A0B4J2B5",
  "term_label": "immunoglobulin mediated immune response",
  "term_id": "GO:0016064",
  "gene_name": "Immunoglobulin heavy variable 3_OR16-9 (non-functional) (Fragment)",
  "gene_symbol": "IGHV3OR16-9"
}